{
  "gene": "UniProtKB:Q8NBT0",
  "term_label": "cilium assembly",
  "gene_symbol": "POC1A",
  "gene_name": "POC1 centriolar protein homolog A",
  "term_id": "GO:0060271"
}